acireductone synthase activity [GO:0043874] (molecular function) Note: This activity is involved in the process of methionine salvage. Sources: RHEA:21700 Relationships: is a type of phosphatase activity [GO:0016791] Definition: Catalysis of the reactions:5-methylsulfanyl-2,3-dioxopentyl phosphate + H2O = 1,2-dihydroxy-5-(methylsulfanyl)pent-1-en-3-one + phosphate. Also known as: E-1 enolase-phosphatase, 5-(methylthio)-2,3-dioxopentyl-phosphate phosphohydrolase (isomerizing), E-1